negative regulation of ephrin receptor signaling pathway [GO:1901188] (biological process) Definition: Any process that stops, prevents or reduces the frequency, rate or extent of ephrin receptor signaling pathway. Sources: GOC:BHF, GOC:TermGenie Also known as: down regulation of Eph receptor signaling pathway, down regulation of Eph receptor signalling pathway, down regulation of ephrin receptor signaling pathway, down-regulation of Eph receptor signaling pathway, down-regulation of Eph receptor signalling pathway, down-regulation of ephrin receptor signaling pathway, downregulation of Eph receptor signaling pathway, downregulation of Eph receptor signalling pathway, downregulation of ephrin receptor signaling pathway, inhibition of Eph receptor signaling pathway, inhibition of Eph receptor signalling pathway, negative regulation of Eph receptor signaling pathway, negative regulation of Eph receptor signalling pathway, inhibition of ephrin receptor signaling pathway Relationships: is a type of negative regulation of signal transduction [GO:0009968]; is a type of regulation of ephrin receptor signaling pathway [GO:1901187]; negatively regulates ephrin receptor signaling pathway [GO:0048013]